{
  "term_label": "cellular response to thyroid hormone stimulus",
  "term_id": "GO:0097067",
  "gene_symbol": "MED1",
  "gene_name": "Mediator of RNA polymerase II transcription subunit 1",
  "gene": "UniProtKB:Q15648"
}